mannogen biosynthetic process [GO:0106304] (biological process) References: PMID:16766650, PMID:31513773, PMID:31662278 Also known as: beta-1,2-mannan biosynthetic process, mannogen anabolism, mannogen biosynthesis, mannogen formation, mannogen synthesis Relationships: is a type of polysaccharide biosynthetic process [GO:0000271] Definition: The chemical reactions and pathways resulting in the formation of mannogen, a mannose-containing polysaccharide that is a major energy reserve in Leishmania.